{
  "term_id": "GO:0046427",
  "gene": "UniProtKB:P22301",
  "term_label": "positive regulation of receptor signaling pathway via JAK-STAT",
  "gene_name": "Interleukin-10",
  "gene_symbol": "IL10"
}